{
  "gene": "UniProtKB:Q9Y6X3",
  "gene_symbol": "MAU2",
  "term_id": "GO:0032116",
  "gene_name": "MAU2 chromatid cohesion factor homolog",
  "term_label": "SMC loading complex"
}